{
  "gene_symbol": "SMIM38",
  "term_id": "UNKNOWN:0003",
  "gene": "UniProtKB:A0A286YFK9",
  "gene_name": "Small integral membrane protein 38",
  "term_label": "Unknown cellular component"
}